{
  "term_label": "Unknown cellular component",
  "gene_name": "NCK-interacting protein with SH3 domain",
  "gene_symbol": "NCKIPSD",
  "term_id": "UNKNOWN:0003",
  "gene": "UniProtKB:Q9NZQ3"
}